{
  "term_id": "UNKNOWN:0001",
  "gene": "UniProtKB:Q9NU02",
  "gene_name": "Ankyrin repeat and EF-hand domain-containing protein 1",
  "gene_symbol": "ANKEF1",
  "term_label": "Unknown molecular function"
}